{
  "gene_name": "Large ribosomal subunit protein eL42",
  "term_label": "cytoplasmic translation",
  "gene": "UniProtKB:P83881",
  "term_id": "GO:0002181",
  "gene_symbol": "RPL36A"
}